{
  "term_label": "RNA polymerase II cis-regulatory region sequence-specific DNA binding",
  "term_id": "GO:0000978",
  "gene": "UniProtKB:Q14814",
  "gene_symbol": "MEF2D",
  "gene_name": "Myocyte-specific enhancer factor 2D"
}